spermidine binding [GO:0019809] (molecular function) Definition: Binding to spermidine, N-(3-aminopropyl)-1,4-diaminobutane. Relationships: is a type of polyamine binding [GO:0019808]; is a type of GO:0043169 Sources: GOC:ai